{
  "gene_name": "Myosin-7",
  "gene": "UniProtKB:P12883",
  "gene_symbol": "MYH7",
  "term_label": "muscle filament sliding",
  "term_id": "GO:0030049"
}